{
  "gene_symbol": "MYADML2",
  "term_id": "UNKNOWN:0001",
  "gene_name": "Myeloid-associated differentiation marker-like protein 2",
  "term_label": "Unknown molecular function",
  "gene": "UniProtKB:A6NDP7"
}